{
  "gene_symbol": "BCL7A",
  "gene": "UniProtKB:Q4VC05",
  "term_label": "Unknown biological process",
  "term_id": "UNKNOWN:0002",
  "gene_name": "B-cell CLL_lymphoma 7 protein family member A"
}